ficolin-1-rich granule lumen [GO:1904813] (cellular component) Also known as: ficolin-1-rich granule membrane-enclosed lumen, membrane-enclosed lumen of ficolin-1 rich granule, membrane-enclosed lumen of ficolin-1-rich granule, membrane-enclosed lumen of ficolin granule Relationships: is a type of intracellular organelle lumen [GO:0070013]; is part of ficolin-1-rich granule [GO:0101002] References: PMID:23650620 Sources: GOC:TermGenie, GO_REF:0000064 Definition: Any membrane-enclosed lumen that is part of a ficolin-1-rich granule.